{
  "gene_name": "Signal transducer and activator of transcription 4",
  "term_id": "GO:0019221",
  "term_label": "cytokine-mediated signaling pathway",
  "gene_symbol": "STAT4",
  "gene": "UniProtKB:Q14765"
}